4-trimethylammoniobutyraldehyde dehydrogenase activity [GO:0047105] (molecular function) Definition: Catalysis of the reaction: NAD+ + 4-trimethylammoniobutanal = NADH + 4-trimethylammoniobutanoate. Sources: EC:1.2.1.47, MetaCyc:1.2.1.47-RXN Also known as: 4-N-trimethylaminobutyraldehyde dehydrogenase activity, 4-trimethylaminobutyraldehyde dehydrogenase activity, 4-trimethylammoniobutanal:NAD+ 1-oxidoreductase activity Relationships: is a type of oxidoreductase activity, acting on the aldehyde or oxo group of donors, NAD or NADP as acceptor [GO:0016620]